{
  "term_label": "Unknown molecular function",
  "term_id": "UNKNOWN:0001",
  "gene_symbol": "OLFML3",
  "gene": "UniProtKB:Q9NRN5",
  "gene_name": "Olfactomedin-like protein 3"
}